mitochondrial valyl-tRNA aminoacylation [GO:0070185] (biological process) Sources: GOC:mah, GOC:mcc Definition: The process of coupling valine to valyl-tRNA in a mitochondrion, catalyzed by valyl-tRNA synthetase. In tRNA aminoacylation, the amino acid is first activated by linkage to AMP and then transferred to either the 2'- or the 3'-hydroxyl group of the 3'-adenosine residue of the tRNA. Relationships: is a type of valyl-tRNA aminoacylation [GO:0006438]; is a type of tRNA aminoacylation for mitochondrial protein translation [GO:0070127]